{
  "gene": "UniProtKB:O00512",
  "gene_name": "B-cell CLL_lymphoma 9 protein",
  "term_label": "beta-catenin binding",
  "gene_symbol": "BCL9",
  "term_id": "GO:0008013"
}